acetyl-CoA C-myristoyltransferase activity [GO:0050633] (molecular function) Sources: EC:2.3.1.155, MetaCyc:2.3.1.155-RXN Relationships: is a type of C-acyltransferase activity [GO:0016408]; is a type of myristoyltransferase activity [GO:0019107] Definition: Catalysis of the reaction: myristoyl-CoA + acetyl-CoA = 3-oxopalmitoyl-CoA + CoA. Also known as: 3-oxopalmitoyl-CoA hydrolase activity, 3-oxopalmitoyl-CoA-CoA acetyltransferase activity, myristoyl-CoA C-acetyltransferase activity, myristoyl-CoA:acetyl-CoA C-myristoyltransferase activity